{
  "gene_symbol": "ZBTB18",
  "gene_name": "Zinc finger and BTB domain-containing protein 18",
  "term_label": "nucleus",
  "term_id": "GO:0005634",
  "gene": "UniProtKB:Q99592"
}